telomere capping [GO:0016233] (biological process) Definition: A process in which telomeres are protected from degradation and fusion, thereby ensuring chromosome stability by protecting the ends from both degradation and from being recognized as damaged DNA. May be mediated by specific single- or double-stranded telomeric DNA binding proteins. References: PMID:11349150, PMID:11352055 Sources: GOC:mah, GOC:rn Also known as: telomere end protection Relationships: is a type of telomere maintenance [GO:0000723] Regulation: regulated by GO:1904353; negatively regulated by GO:1904354; RO_0002213 by positive regulation of telomere capping [GO:1904355]